{
  "gene_name": "cAMP-dependent protein kinase catalytic subunit gamma",
  "gene": "UniProtKB:P22612",
  "term_label": "nucleus",
  "gene_symbol": "PRKACG",
  "term_id": "GO:0005634"
}